{
  "gene": "UniProtKB:Q6ZSG1",
  "gene_name": "E3 ubiquitin-protein ligase ARK2C",
  "gene_symbol": "ARK2C",
  "term_label": "positive regulation of BMP signaling pathway",
  "term_id": "GO:0030513"
}